{
  "gene": "UniProtKB:O60741",
  "gene_symbol": "HCN1",
  "term_id": "GO:0071805",
  "term_label": "potassium ion transmembrane transport",
  "gene_name": "Potassium_sodium hyperpolarization-activated cyclic nucleotide-gated channel 1"
}